proteolysis involved in protein catabolic process [GO:0051603] (biological process) Relationships: is a type of proteolysis [GO:0006508]; is part of protein catabolic process [GO:0030163] Definition: The hydrolysis of a peptide bond or bonds within a protein as part of the chemical reactions and pathways resulting in the breakdown of a protein by individual cells. Also known as: peptidolysis involved in cellular protein catabolic process, peptidolysis involved in cellular protein catabolism, proteolysis involved in cellular protein catabolic process, peptidolysis during cellular protein catabolic process, peptidolysis during cellular protein catabolism, proteolysis during cellular protein catabolic process, proteolysis during cellular protein catabolism Sources: GOC:ai, GOC:dph, GOC:tb Subtypes: GO:0002077, proteolysis associated with antigen processing and presentation [GO:0002496], protein quality control for misfolded or incompletely synthesized proteins [GO:0006515], proteasomal protein catabolic process [GO:0010498], modification-dependent protein catabolic process [GO:0019941], ubiquitin-independent protein catabolic process via the multivesicular body sorting pathway [GO:0090611], membrane protein proteolysis involved in retrograde protein transport, ER to cytosol [GO:1904211] Regulation: regulated by regulation of proteolysis involved in protein catabolic process [GO:1903050]; negatively regulated by negative regulation of proteolysis involved in protein catabolic process [GO:1903051]; positively regulated by GO:1903052